{
  "term_id": "UNKNOWN:0003",
  "gene_name": "Inositol polyphosphate-5-phosphatase A",
  "gene": "UniProtKB:Q14642",
  "gene_symbol": "INPP5A",
  "term_label": "Unknown cellular component"
}